fucose metabolic process [GO:0006004] (biological process) Sources: ISBN:0198506732 Relationships: is a type of hexose metabolic process [GO:0019318] Also known as: fucose metabolism Subtypes: fucose catabolic process [GO:0019317], fucose biosynthetic process [GO:0042353], L-fucose metabolic process [GO:0042354] Definition: The chemical reactions and pathways involving fucose, or 6-deoxygalactose, which has two enantiomers, D-fucose and L-fucose.